{
  "gene": "UniProtKB:Q9Y2B1",
  "gene_symbol": "RXYLT1",
  "gene_name": "Ribitol-5-phosphate xylosyltransferase 1",
  "term_label": "ribitol beta-1,4-xylosyltransferase activity",
  "term_id": "GO:0120053"
}